{
  "gene_name": "Rhotekin-2",
  "term_id": "UNKNOWN:0001",
  "term_label": "Unknown molecular function",
  "gene_symbol": "RTKN2",
  "gene": "UniProtKB:Q8IZC4"
}